{
  "gene_name": "B-cell receptor CD22",
  "term_id": "GO:0009897",
  "gene": "UniProtKB:P20273",
  "term_label": "external side of plasma membrane",
  "gene_symbol": "CD22"
}